{
  "gene_symbol": "APC",
  "term_label": "nervous system development",
  "gene_name": "Adenomatous polyposis coli protein",
  "term_id": "GO:0007399",
  "gene": "UniProtKB:P25054"
}